{
  "term_id": "UNKNOWN:0003",
  "gene_symbol": "FBXO46",
  "gene": "UniProtKB:Q6PJ61",
  "gene_name": "F-box only protein 46",
  "term_label": "Unknown cellular component"
}